{
  "term_label": "calcium export from the mitochondrion",
  "gene_symbol": "SLC8B1",
  "term_id": "GO:0099093",
  "gene_name": "Mitochondrial sodium_calcium exchanger protein",
  "gene": "UniProtKB:Q6J4K2"
}